positive regulation of chondrocyte differentiation [GO:0032332] (biological process) Definition: Any process that activates or increases the frequency, rate or extent of chondrocyte differentiation. Also known as: up regulation of chondrocyte differentiation, up-regulation of chondrocyte differentiation, upregulation of chondrocyte differentiation, activation of chondrocyte differentiation, stimulation of chondrocyte differentiation Sources: GOC:mah Relationships: is a type of GO:0032330; is a type of GO:0045597; is a type of positive regulation of cartilage development [GO:0061036]; positively regulates chondrocyte differentiation [GO:0002062] Subtypes: positive regulation of chondrocyte development [GO:1902761]